{
  "term_label": "intracellular iron ion homeostasis",
  "gene": "UniProtKB:Q9NZ45",
  "term_id": "GO:0006879",
  "gene_symbol": "CISD1",
  "gene_name": "CDGSH iron-sulfur domain-containing protein 1"
}